{
  "gene": "UniProtKB:P10915",
  "gene_name": "Hyaluronan and proteoglycan link protein 1",
  "term_id": "GO:0045202",
  "gene_symbol": "HAPLN1",
  "term_label": "synapse"
}